{
  "gene": "UniProtKB:Q08708",
  "term_label": "plasma membrane",
  "gene_symbol": "CD300C",
  "term_id": "GO:0005886",
  "gene_name": "CMRF35-like molecule 6"
}